{
  "term_label": "microtubule",
  "term_id": "GO:0005874",
  "gene_name": "Kinesin-like protein KIF17",
  "gene_symbol": "KIF17",
  "gene": "UniProtKB:Q9P2E2"
}